{
  "gene_symbol": "CNGA1",
  "term_label": "plasma membrane",
  "gene_name": "cGMP-gated cation channel alpha-1",
  "term_id": "GO:0005886",
  "gene": "UniProtKB:P29973"
}